{
  "gene_symbol": "NID1",
  "term_label": "Unknown molecular function",
  "gene_name": "Nidogen-1",
  "gene": "UniProtKB:P14543",
  "term_id": "UNKNOWN:0001"
}